regulation of metanephros development [GO:0072215] (biological process) Definition: Any process that modulates the rate, frequency or extent of metanephros development. Metanephros development is the process whose specific outcome is the progression of the metanephros over time, from its formation to the mature structure. The metanephros is an endocrine and metabolic organ that filters the blood and excretes the end products of body metabolism in the form of urine. Relationships: is a type of regulation of kidney development [GO:0090183]; regulates metanephros development [GO:0001656] Sources: GOC:mtg_kidney_jan10 Subtypes: positive regulation of metanephros development [GO:0072216], GO:0072217, GO:2001074